host cell nucleolus [GO:0044196] (cellular component) Definition: A small, dense body one or more of which are present in the nucleus of eukaryotic host cells. Relationships: is a type of GO:0044094 Sources: GOC:jl